regulation of amyloid precursor protein catabolic process [GO:1902991] (biological process) Definition: Any process that modulates the frequency, rate or extent of amyloid precursor protein catabolic process. References: PMID:24499793 Sources: GOC:PARL, GOC:TermGenie, GOC:rl, GO_REF:0000058 Note: An example of this is human FKBP1A/12 (UniProt symbol P62942) in PMID:24499793 (inferred from direct assay). Relationships: is_a regulation of protein metabolic process [GO:0051246]; regulates GO:0042987 Subtypes: regulation of amyloid-beta formation [GO:1902003], negative regulation of amyloid precursor protein catabolic process [GO:1902992], positive regulation of amyloid precursor protein catabolic process [GO:1902993] Also known as: regulation of APP catabolic process, regulation of APP catabolism, regulation of amyloid precursor protein breakdown, regulation of amyloid precursor protein catabolism, regulation of amyloid precursor protein degradation